{
  "gene_symbol": "C2orf92",
  "gene": "UniProtKB:A0A1B0GVN3",
  "term_id": "UNKNOWN:0001",
  "gene_name": "Uncharacterized protein C2orf92",
  "term_label": "Unknown molecular function"
}